poly(glycerol phosphate) teichoic acid biosynthetic process [GO:1902014] (biological process) Definition: The chemical reactions and pathways resulting in the formation of poly(glycerol phosphate) teichoic acid. Also known as: poly(glycerol phosphate) teichoic acid anabolism, poly(glycerol phosphate) teichoic acid biosynthesis, poly(glycerol phosphate) teichoic acid formation, poly(glycerol phosphate) teichoic acid synthesis References: PMID:11882717 Sources: GOC:TermGenie, UniPathway:UPA00827 Relationships: is a type of teichoic acid biosynthetic process [GO:0019350]